{
  "gene": "UniProtKB:Q13445",
  "term_label": "Golgi organization",
  "gene_name": "Transmembrane emp24 domain-containing protein 1",
  "term_id": "GO:0007030",
  "gene_symbol": "TMED1"
}